{
  "term_label": "extracellular space",
  "gene_symbol": "CCL7",
  "gene_name": "C-C motif chemokine 7",
  "gene": "UniProtKB:P80098",
  "term_id": "GO:0005615"
}